inner dynein arm [GO:0036156] (CC) Definition: Inner arm structure present on the outer doublet microtubules of ciliary and flagellar axonemes. The structure of inner dynein arms is complex and may vary within the axoneme. Inner dynein arms are heteromeric, comprising 8 different heavy chains and various subunits. Inner and outer dynein arms have different functions in the generation of microtubule-based motility. Relationships: is a type of axonemal dynein complex [GO:0005858] References: PMID:19347929, PMID:2557057, PMID:7962092 Sources: GOC:BHF, GOC:vk Also known as: inner dynein arm complex